D-iditol 2-dehydrogenase activity [GO:0047824] (molecular function) Sources: RHEA:12725 Definition: Catalysis of the reaction: D-iditol + NAD+ = D-sorbose + NADH. Relationships: is a type of oxidoreductase activity, acting on the CH-OH group of donors, NAD or NADP as acceptor [GO:0016616]; is a type of hexitol dehydrogenase activity [GO:0031320]